{
  "gene": "UniProtKB:Q8N8U3",
  "term_id": "UNKNOWN:0002",
  "gene_name": "Retrotransposon Gag-like protein 3",
  "term_label": "Unknown biological process",
  "gene_symbol": "RTL3"
}